{
  "gene": "UniProtKB:Q9BUV0",
  "term_id": "UNKNOWN:0003",
  "gene_symbol": "RSRP1",
  "term_label": "Unknown cellular component",
  "gene_name": "Arginine_serine-rich protein 1"
}